{
  "gene_name": "Small ubiquitin-related modifier 1",
  "gene": "UniProtKB:P63165",
  "term_id": "GO:0044389",
  "term_label": "ubiquitin-like protein ligase binding",
  "gene_symbol": "SUMO1"
}